{
  "gene_name": "Signaling lymphocytic activation molecule",
  "term_label": "signaling receptor activity",
  "gene_symbol": "SLAMF1",
  "term_id": "GO:0038023",
  "gene": "UniProtKB:Q13291"
}